positive regulation of response to reactive oxygen species [GO:1901033] (biological process) Relationships: is a type of regulation of response to reactive oxygen species [GO:1901031]; is a type of GO:1902884; positively regulates response to reactive oxygen species [GO:0000302] Definition: Any process that activates or increases the frequency, rate or extent of response to reactive oxygen species. Also known as: activation of response to AOS, activation of response to ROI, activation of response to ROS, activation of response to active oxygen species, activation of response to reactive oxidative species, activation of response to reactive oxygen intermediate, positive regulation of response to AOS, positive regulation of response to ROI, positive regulation of response to ROS, positive regulation of response to active oxygen species, positive regulation of response to reactive oxidative species, positive regulation of response to reactive oxygen intermediate, up regulation of response to AOS, up regulation of response to ROI, up regulation of response to ROS, up regulation of response to active oxygen species, up regulation of response to reactive oxidative species, up regulation of response to reactive oxygen intermediate, up regulation of response to reactive oxygen species, up-regulation of response to AOS, up-regulation of response to ROI, up-regulation of response to ROS, up-regulation of response to active oxygen species, up-regulation of response to reactive oxidative species, up-regulation of response to reactive oxygen intermediate, up-regulation of response to reactive oxygen species, upregulation of response to AOS, upregulation of response to ROI, upregulation of response to ROS, upregulation of response to active oxygen species, upregulation of response to reactive oxidative species, upregulation of response to reactive oxygen intermediate, upregulation of response to reactive oxygen species, activation of response to reactive oxygen species Sources: GOC:TermGenie, GOC:kmv